{
  "term_label": "cytoplasm",
  "gene_symbol": "ANKHD1",
  "gene": "UniProtKB:Q8IWZ3",
  "term_id": "GO:0005737",
  "gene_name": "Ankyrin repeat and KH domain-containing protein 1"
}